{
  "term_label": "perinuclear region of cytoplasm",
  "gene_name": "Protein S100-A4",
  "gene_symbol": "S100A4",
  "term_id": "GO:0048471",
  "gene": "UniProtKB:P26447"
}